surface biofilm formation [GO:0090604] (biological process) Relationships: is a type of biofilm formation [GO:0042710] Subtypes: GO:0090606 Sources: GOC:di, GOC:tb Definition: A process in which planktonically growing microorganisms grow at the surface of a liquid-air interface and produce extracellular polymers that facilitate matrix formation, resulting in a change in the organisms' growth rate and gene transcription.